{
  "term_label": "acetylglucosaminyltransferase activity",
  "gene_symbol": "MGAT4D",
  "term_id": "GO:0008375",
  "gene": "UniProtKB:A6NG13",
  "gene_name": "Alpha-1,3-mannosyl-glycoprotein 4-beta-N-acetylglucosaminyltransferase-like protein MGAT4D"
}